{
  "term_id": "GO:0007216",
  "gene": "UniProtKB:P41594",
  "term_label": "G protein-coupled glutamate receptor signaling pathway",
  "gene_name": "Metabotropic glutamate receptor 5",
  "gene_symbol": "GRM5"
}